{
  "gene_name": "Protein odd-skipped-related 2",
  "term_id": "GO:0000981",
  "term_label": "DNA-binding transcription factor activity, RNA polymerase II-specific",
  "gene": "UniProtKB:Q8N2R0",
  "gene_symbol": "OSR2"
}